{
  "term_id": "GO:0038203",
  "gene_name": "Target of rapamycin complex 2 subunit MAPKAP1",
  "term_label": "TORC2 signaling",
  "gene": "UniProtKB:Q9BPZ7",
  "gene_symbol": "MAPKAP1"
}